bile acid conjugation [GO:0002152] (biological process) Note: The bile acid is first activated using CoA by cholate-CoA ligase activity(GO:0047747), then conjugated to taurine or glycine by glycine N-choloyltransferase activity (GO:0047963; appears to use either glycine or taurine). References: PMID:1094911, PMID:708413 Definition: The process in which bile acids are covalently linked to taurine or glycine. Relationships: is a type of bile acid metabolic process [GO:0008206]